deSUMOylase activity [GO:0016929] (molecular function) Also known as: SUMO-specific isopeptidase activity, SUMO-specific protease activity, SUSP, ULP References: PMID:10094048, PMID:11031248, PMID:11265250, PMID:23746258 Sources: GOC:rn Definition: An thiol-dependent isopeptidase activity that cleaves SUMO from a target protein to which it is conjugated. Relationships: is a type of cysteine-type peptidase activity [GO:0008234]; is a type of ubiquitin-like protein peptidase activity [GO:0019783]